{
  "gene_name": "Transmembrane protein 178B",
  "term_label": "membrane",
  "gene": "UniProtKB:H3BS89",
  "term_id": "GO:0016020",
  "gene_symbol": "TMEM178B"
}